{
  "gene": "UniProtKB:Q7Z4S6",
  "term_label": "ATP hydrolysis activity",
  "term_id": "GO:0016887",
  "gene_name": "Kinesin-like protein KIF21A",
  "gene_symbol": "KIF21A"
}